{
  "term_id": "GO:0017154",
  "gene_name": "Neuropilin-1",
  "term_label": "semaphorin receptor activity",
  "gene_symbol": "NRP1",
  "gene": "UniProtKB:O14786"
}